{
  "gene": "UniProtKB:Q9H2S9",
  "gene_symbol": "IKZF4",
  "term_label": "regulation of transcription by RNA polymerase II",
  "gene_name": "Zinc finger protein Eos",
  "term_id": "GO:0006357"
}